{
  "term_id": "GO:0005549",
  "gene": "UniProtKB:Q8NGQ4",
  "term_label": "odorant binding",
  "gene_symbol": "OR10Q1",
  "gene_name": "Olfactory receptor 10Q1"
}